{
  "gene": "UniProtKB:O94916",
  "term_label": "DNA-binding transcription factor activity, RNA polymerase II-specific",
  "term_id": "GO:0000981",
  "gene_symbol": "NFAT5",
  "gene_name": "Nuclear factor of activated T-cells 5"
}